{
  "term_id": "GO:0031410",
  "gene_name": "Rho-related BTB domain-containing protein 1",
  "gene": "UniProtKB:O94844",
  "gene_symbol": "RHOBTB1",
  "term_label": "cytoplasmic vesicle"
}